conus arteriosus development [GO:0003238] (biological process) Sources: GOC:mtg_heart Definition: The progression of the conus arteriosus over time, from its formation to the mature structure. The conus arteriosus is a valved chamber with thick muscular walls stemming from the ventricle and connecting to the pulmonary trunk. Relationships: is a type of cardiac chamber development [GO:0003205]